{
  "term_id": "GO:0002323",
  "gene": "UniProtKB:Q9BZW8",
  "term_label": "natural killer cell activation involved in immune response",
  "gene_name": "Natural killer cell receptor 2B4",
  "gene_symbol": "CD244"
}